{
  "term_id": "GO:0005829",
  "term_label": "cytosol",
  "gene": "UniProtKB:O77932",
  "gene_name": "Decapping and exoribonuclease protein",
  "gene_symbol": "DXO"
}